{
  "term_label": "modulation of chemical synaptic transmission",
  "gene": "UniProtKB:P01138",
  "gene_symbol": "NGF",
  "gene_name": "Beta-nerve growth factor",
  "term_id": "GO:0050804"
}